{
  "gene_name": "Amelotin",
  "gene_symbol": "AMTN",
  "gene": "UniProtKB:Q6UX39",
  "term_label": "basement membrane",
  "term_id": "GO:0005604"
}